{
  "term_label": "cholesterol transfer activity",
  "gene_name": "Apolipoprotein A-I",
  "term_id": "GO:0120020",
  "gene_symbol": "APOA1",
  "gene": "UniProtKB:P02647"
}